{
  "gene_name": "FACT complex subunit SPT16",
  "gene_symbol": "SUPT16H",
  "gene": "UniProtKB:Q9Y5B9",
  "term_id": "GO:0035101",
  "term_label": "FACT complex"
}